dendritic transport of ribonucleoprotein complex [GO:0098961] (biological process) Also known as: dendritic transport of RNP complex Definition: The directed movement of a ribonucleoprotein complex along microtubules in nerve cell dendrites. Sources: GOC:dos Relationships: is a type of dendritic transport [GO:0098935]; occurs in dendrite cytoplasm [GO:0032839]